{
  "term_id": "UNKNOWN:0001",
  "gene_name": "N-cym protein",
  "gene_symbol": "MYCNOS",
  "gene": "UniProtKB:P40205",
  "term_label": "Unknown molecular function"
}